{
  "gene_name": "Jhy protein homolog",
  "gene": "UniProtKB:Q6NUN7",
  "term_label": "Unknown molecular function",
  "gene_symbol": "JHY",
  "term_id": "UNKNOWN:0001"
}